{
  "term_id": "GO:0003730",
  "gene_name": "Heterogeneous nuclear ribonucleoproteins A2_B1",
  "gene": "UniProtKB:P22626",
  "term_label": "mRNA 3'-UTR binding",
  "gene_symbol": "HNRNPA2B1"
}